{
  "gene_symbol": "OR4M2",
  "gene": "UniProtKB:Q8NGB6",
  "gene_name": "Olfactory receptor 4M2",
  "term_label": "Unknown biological process",
  "term_id": "UNKNOWN:0002"
}